{
  "term_id": "UNKNOWN:0003",
  "gene_symbol": "TRAJ61",
  "gene_name": "T cell receptor alpha joining 61 (non-functional) (Fragment)",
  "term_label": "Unknown cellular component",
  "gene": "UniProtKB:A0A075B708"
}